{
  "gene_name": "Semaphorin-3F",
  "gene_symbol": "SEMA3F",
  "term_id": "GO:0050919",
  "gene": "UniProtKB:Q13275",
  "term_label": "negative chemotaxis"
}